mucilage pectin metabolic process [GO:0048363] (biological process) Sources: GOC:jid Definition: The chemical reactions and pathways involving the pectin component of mucilage. Subtypes: mucilage pectin biosynthetic process [GO:0048358] Also known as: mucilage pectin metabolism Relationships: is a type of pectin metabolic process [GO:0045488]